{
  "gene_symbol": "YIF1B",
  "gene_name": "Protein YIF1B",
  "term_id": "GO:0000139",
  "gene": "UniProtKB:Q5BJH7",
  "term_label": "Golgi membrane"
}